4-chlorobiphenyl metabolic process [GO:0018880] (biological process) Definition: The chemical reactions and pathways involving 4-chlorobiphenyl, a member of the polychlorinated biphenyl (PCB) group of compounds, a very stable group of synthetic organic compounds composed of a biphenyl nucleus with 1-10 chlorine substituents. 4-chlorobiphenyl has been used as a model substrate to investigate PCB degradation. Relationships: is a type of GO:0042197; is a type of GO:0042537 Sources: GOC:jl Also known as: 4-chlorobiphenyl metabolism